{
  "gene_name": "Inositol monophosphatase 1",
  "gene_symbol": "IMPA1",
  "term_label": "inositol metabolic process",
  "gene": "UniProtKB:P29218",
  "term_id": "GO:0006020"
}